{
  "gene_name": "Cylicin-2",
  "term_id": "UNKNOWN:0002",
  "term_label": "Unknown biological process",
  "gene_symbol": "CYLC2",
  "gene": "UniProtKB:Q14093"
}